{
  "gene_symbol": "ZKSCAN2",
  "term_id": "GO:0006357",
  "gene_name": "Zinc finger protein with KRAB and SCAN domains 2",
  "gene": "UniProtKB:Q63HK3",
  "term_label": "regulation of transcription by RNA polymerase II"
}